{
  "gene_name": "Guanine nucleotide-binding protein G(q) subunit alpha",
  "term_id": "GO:0005834",
  "gene_symbol": "GNAQ",
  "term_label": "heterotrimeric G-protein complex",
  "gene": "UniProtKB:P50148"
}